{
  "term_id": "UNKNOWN:0001",
  "gene_name": "Netrin receptor DCC",
  "gene_symbol": "DCC",
  "term_label": "Unknown molecular function",
  "gene": "UniProtKB:P43146"
}